tRNA (guanine(10)-N2)-dimethyltransferase activity [GO:0160101] (molecular function) Definition: Catalysis of the reaction: guanosine(10) in tRNA + 2 S-adenosyl-L-methionine = 2 H+ + N(2)-dimethylguanosine(10) in tRNA + 2 S-adenosyl-L-homocysteine. Relationships: is a type of N-methyltransferase activity [GO:0008170]; is_a GO:0016423 Sources: EC:2.1.1.213 Also known as: N(2),N(2)-dimethylguanosine tRNA methyltransferase, tRNA (guanine(10)-N(2))-dimethyltransferase activity, tRNA (guanosine(10)-N(2))-dimethyltransferase activity